{
  "gene_symbol": "MAP2K5",
  "term_label": "Unknown cellular component",
  "term_id": "UNKNOWN:0003",
  "gene": "UniProtKB:Q13163",
  "gene_name": "Dual specificity mitogen-activated protein kinase kinase 5"
}